{
  "gene_symbol": "GPR108",
  "term_id": "GO:0016020",
  "gene": "UniProtKB:Q9NPR9",
  "gene_name": "Protein GPR108",
  "term_label": "membrane"
}